regulation of high-density lipoprotein particle assembly [GO:0090107] (biological process) Definition: Any process that modulates the frequency, rate, or extent of high-density lipoprotein particle assembly. High-density lipoprotein particle assembly is the aggregation and arrangement of proteins and lipids to form a high-density lipoprotein particle. Relationships: is a type of regulation of protein-containing complex assembly [GO:0043254]; is a type of regulation of multicellular organismal process [GO:0051239]; regulates GO:0034380 Subtypes: positive regulation of high-density lipoprotein particle assembly [GO:0090108] Sources: GOC:dph, GOC:tb